{
  "term_id": "UNKNOWN:0001",
  "gene_name": "Sperm-associated antigen 11A",
  "gene_symbol": "SPAG11A",
  "term_label": "Unknown molecular function",
  "gene": "UniProtKB:Q6PDA7"
}